{
  "term_label": "cytoplasm",
  "gene_name": "SERPINE1 mRNA-binding protein 1",
  "term_id": "GO:0005737",
  "gene": "UniProtKB:Q8NC51",
  "gene_symbol": "SERBP1"
}